positive regulation of metanephric cap mesenchymal cell proliferation [GO:0090096] (biological process) Sources: GOC:dph, GOC:tb, GOC:yaf Definition: Any process that increases the frequency, rate, or extent of metanephric cap mesenchymal cell proliferation. Metanephric cap mesenchymal cell proliferation is the multiplication or reproduction of metanephric cap mesenchymal cells, resulting in the expansion of the cell population. A metanephric cap mesenchymal cell is a mesenchymal cell that has condensed with other mesenchymal cells surrounding the ureteric bud tip. Relationships: is a type of positive regulation of mesenchymal cell proliferation [GO:0002053]; is a type of regulation of metanephric cap mesenchymal cell proliferation [GO:0090095]; is a type of positive regulation of kidney development [GO:0090184]; is a type of positive regulation of cell proliferation involved in kidney development [GO:1901724]; positively regulates metanephric cap mesenchymal cell proliferation involved in metanephros development [GO:0090094]